{
  "gene_symbol": "PARG",
  "gene": "UniProtKB:Q86W56",
  "gene_name": "Poly(ADP-ribose) glycohydrolase",
  "term_id": "GO:0005634",
  "term_label": "nucleus"
}